benzoate transmembrane transporter activity [GO:0042925] (molecular function) Sources: GOC:jl, ISBN:0721662544 Also known as: benzoate transporter activity Relationships: is a type of xenobiotic transmembrane transporter activity [GO:0042910]; is a type of carboxylic acid transmembrane transporter activity [GO:0046943]; is part of GO:0042919 Definition: Enables the directed movement of benzoate, the anion of benzoic acid (benzenecarboxylic acid) from one side of a membrane to the other.